adherens junction [GO:0005912] (CC) Subtypes: spot adherens junction [GO:0005914], zonula adherens [GO:0005915] Relationships: is a type of cell-cell junction [GO:0005911] References: PMID:17854762, PMID:20571587, PMID:21422226, PMID:28096264 Sources: GOC:aruk, GOC:bc, GOC:mah, ISBN:0198506732 Definition: A cell-cell junction composed of the epithelial cadherin-catenin complex. The epithelial cadherins, or E-cadherins, of each interacting cell extend through the plasma membrane into the extracellular space and bind to each other. The E-cadherins bind to catenins on the cytoplasmic side of the membrane, where the E-cadherin-catenin complex binds to cytoskeletal components and regulatory and signaling molecules. Also known as: cell-cell adherens junction